succinate import across plasma membrane [GO:0098720] (biological process) Sources: GOC:dos Definition: The directed movement of succinate from outside of a cell, across the plasma membrane and into the cytosol. Relationships: is a type of GO:0071422; is_a import across plasma membrane [GO:0098739] Also known as: succinate import into cell